reciprocal meiotic recombination [GO:0007131] (biological process) Regulation: regulated by regulation of reciprocal meiotic recombination [GO:0010520]; positively regulated by positive regulation of reciprocal meiotic recombination [GO:0010845]; negatively regulated by GO:0045128 Relationships: is a type of GO:0140527; is a type of meiotic cell cycle process [GO:1903046]; is part of meiosis I [GO:0007127] References: PMID:2087779 Also known as: gene conversion with reciprocal crossover, female meiotic recombination Definition: The cell cycle process in which double strand breaks are formed and repaired through a single or double Holliday junction intermediate. This results in the equal exchange of genetic material between non-sister chromatids in a pair of homologous chromosomes. These reciprocal recombinant products ensure the proper segregation of homologous chromosomes during meiosis I and create genetic diversity.